{
  "gene_symbol": "H1-10",
  "gene_name": "Histone H1.10",
  "term_id": "GO:0045910",
  "term_label": "negative regulation of DNA recombination",
  "gene": "UniProtKB:Q92522"
}